positive regulation of integrin-mediated signaling pathway [GO:2001046] (biological process) Sources: GOC:obol Relationships: is_a positive regulation of signal transduction [GO:0009967]; is a type of GO:2001044; positively regulates integrin-mediated signaling pathway [GO:0007229] Definition: Any process that activates or increases the frequency, rate or extent of integrin-mediated signaling pathway. Also known as: positive regulation of integrin-mediated signalling pathway